{
  "gene": "UniProtKB:O14981",
  "gene_symbol": "BTAF1",
  "term_id": "UNKNOWN:0001",
  "term_label": "Unknown molecular function",
  "gene_name": "TATA-binding protein-associated factor 172"
}